fibroblast growth factor receptor signaling pathway [GO:0008543] (biological process) Relationships: is_a cell surface receptor protein tyrosine kinase signaling pathway [GO:0007169]; is part of cellular response to fibroblast growth factor stimulus [GO:0044344] Regulation: RO_0002211 by regulation of fibroblast growth factor receptor signaling pathway [GO:0040036]; negatively regulated by negative regulation of fibroblast growth factor receptor signaling pathway [GO:0040037]; positively regulated by GO:0045743 Subtypes: GO:0021875, GO:0021899, fibroblast growth factor receptor signaling pathway involved in spinal cord anterior/posterior pattern formation [GO:0021907], fibroblast growth factor receptor signaling pathway involved in negative regulation of apoptotic process in bone marrow cell [GO:0035602], fibroblast growth factor receptor signaling pathway involved in hemopoiesis [GO:0035603], fibroblast growth factor receptor signaling pathway involved in positive regulation of cell proliferation in bone marrow [GO:0035604], fibroblast growth factor receptor signaling pathway involved in orbitofrontal cortex development [GO:0035607], fibroblast growth factor receptor signaling pathway involved in mammary gland specification [GO:0060595], GO:0060787, fibroblast growth factor receptor signaling pathway involved in neural plate anterior/posterior pattern formation [GO:0060825], fibroblast growth factor receptor signaling pathway involved in heart development [GO:0061313], GO:0090080, fibroblast growth factor receptor signaling pathway involved in somitogenesis [GO:0090243], GO:1902178, fibroblast growth factor receptor signaling pathway involved in ureteric bud formation [GO:2000699] Also known as: FGF receptor signaling pathway, FGF receptor signalling pathway, FGFR signaling pathway, fibroblast growth factor receptor signalling pathway Definition: The series of molecular signals generated as a consequence of a fibroblast growth factor receptor binding to one of its physiological ligands. Sources: GOC:ceb